{
  "gene_symbol": "LINC01556",
  "term_label": "Unknown cellular component",
  "gene": "UniProtKB:Q5JQF7",
  "gene_name": "Putative uncharacterized protein encoded by LINC01556",
  "term_id": "UNKNOWN:0003"
}